{
  "term_label": "Unknown cellular component",
  "gene_name": "Immunoglobulin heavy variable 3-9",
  "term_id": "UNKNOWN:0003",
  "gene": "UniProtKB:P01782",
  "gene_symbol": "IGHV3-9"
}